activin secretion [GO:0032333] (biological process) Sources: GOC:mah Regulation: regulated by regulation of activin secretion [GO:0032335]; negatively regulated by negative regulation of activin secretion [GO:0032336]; positively regulated by positive regulation of activin secretion [GO:0032337] Relationships: is a type of hormone secretion [GO:0046879] Definition: The regulated release of activin, a nonsteroidal regulator composed of two covalently linked beta subunits, which is synthesized in the pituitary gland and gonads and stimulates the secretion of follicle-stimulating hormone.